{
  "gene_symbol": "CENPH",
  "gene_name": "Centromere protein H",
  "term_label": "kinetochore",
  "term_id": "GO:0000776",
  "gene": "UniProtKB:Q9H3R5"
}